axial mesoderm structural organization [GO:0048331] (biological process) Also known as: axial mesoderm structural organisation Relationships: is a type of mesoderm structural organization [GO:0048338]; BFO_0000050 axial mesoderm morphogenesis [GO:0048319] Sources: GOC:dgh Definition: The process that contributes to the act of creating the structural organization of the axial mesoderm. This process pertains to the physical shaping of a rudimentary structure.